{
  "gene_name": "Apolipoprotein A-V",
  "term_id": "GO:0034364",
  "term_label": "high-density lipoprotein particle",
  "gene_symbol": "APOA5",
  "gene": "UniProtKB:Q6Q788"
}